homocysteine desulfhydrase activity [GO:0047982] (molecular function) Sources: EC:4.4.1.2, MetaCyc:HOMOCYSTEINE-DESULFHYDRASE-RXN Relationships: is a type of carbon-sulfur lyase activity [GO:0016846] Definition: Catalysis of the reaction: L-homocysteine + H2O = sulfide + NH3 + 2-oxobutanoate. Also known as: L-homocysteine hydrogen-sulfide-lyase (deaminating), L-homocysteine hydrogen-sulfide-lyase (deaminating; 2-oxobutanoate-forming), homocysteine desulfurase activity